omegasome membrane [GO:1903349] (cellular component) Relationships: is a type of bounding membrane of organelle [GO:0098588]; is part of GO:1990462 Definition: Any membrane that is part of an omegasome. References: PMID:18725538, PMID:24591649 Sources: GOC:TermGenie, GOC:mf, GO_REF:0000064